hydrolase activity, acting on acid halide bonds [GO:0016824] (molecular function) Definition: Catalysis of the hydrolysis of any acid halide bond. Relationships: is a type of hydrolase activity [GO:0016787] Sources: EC:3.8.-.- Subtypes: GO:0019120, GO:0047862